{
  "term_id": "UNKNOWN:0002",
  "term_label": "Unknown biological process",
  "gene_name": "Fer-1-like protein 4",
  "gene": "UniProtKB:A9Z1Z3",
  "gene_symbol": "FER1L4"
}